ubiquitin ligase inhibitor activity [GO:1990948] (molecular function) References: PMID:21389117 Sources: GOC:dph, GOC:vw Relationships: is a type of ubiquitin-protein transferase inhibitor activity [GO:0055105] Also known as: APC-Cdc20 complex inhibitor activity, mitotic anaphase-promoting complex inhibitor activity Definition: Binds to and stops, prevents or reduces the activity of a ubiquitin ligase.